{
  "term_id": "GO:0006357",
  "gene": "UniProtKB:Q99612",
  "gene_name": "Krueppel-like factor 6",
  "term_label": "regulation of transcription by RNA polymerase II",
  "gene_symbol": "KLF6"
}